U2-type catalytic step 2 spliceosome [GO:0071007] (cellular component) Definition: A spliceosomal complex that contains the U2, U5 and U6 snRNPs bound to a splicing intermediate in which the first catalytic cleavage of the 5' splice site has occurred. The precise subunit composition differs significantly from that of the catalytic step 1, or activated, spliceosome, and includes many proteins in addition to those found in the U2, U5 and U6 snRNPs. References: PMID:18322460, PMID:19239890 Sources: GOC:ab, GOC:krc, GOC:mah, ISBN:0879695897, ISBN:0879697393 Also known as: major catalytic step 2 spliceosome, GT-AG catalytic step 2 spliceosome, mammalian U2-type spliceosomal complex C, mammalian U2-type spliceosomal complex C1, yeast U2-type spliceosomal complex A2-2 Relationships: is a type of U2-type spliceosomal complex [GO:0005684]; is a type of GO:0071013; BFO_0000051 U2 snRNP [GO:0005686]; has part U6 snRNP [GO:0005688]